response to erythropoietin [GO:0036017] (biological process) Definition: Any process that results in a change in state or activity of a cell or an organism (in terms of movement, secretion, enzyme production, gene expression, etc.) as a result of an erythropoietin stimulus. Erythropoietin is a glycoprotein hormone that controls erythropoiesis. Sources: GOC:yaf Relationships: is a type of GO:0034097 Subtypes: cellular response to erythropoietin [GO:0036018]